{
  "gene": "UniProtKB:Q7Z794",
  "term_label": "keratin filament",
  "gene_symbol": "KRT77",
  "term_id": "GO:0045095",
  "gene_name": "Keratin, type II cytoskeletal 1b"
}